{
  "gene": "UniProtKB:O00421",
  "term_id": "GO:0016493",
  "gene_name": "C-C chemokine receptor-like 2",
  "term_label": "C-C chemokine receptor activity",
  "gene_symbol": "CCRL2"
}